Notch signaling pathway involved in forebrain neuroblast division [GO:0021876] (biological process) Also known as: Notch signalling pathway in forebrain neuroblast division Definition: The series of molecular signals initiated by binding of an extracellular ligand to a Notch receptor on the surface of the target cell that contributes to the self renewal of neuroblasts in the forebrain. Relationships: is_a GO:0007219; is part of forebrain neuroblast division [GO:0021873] References: PMID:16226447 Sources: GOC:cls, GOC:dgh, GOC:dph, GOC:jid, GO_REF:0000021